regulation of interleukin-19 production [GO:0032662] (biological process) Definition: Any process that modulates the frequency, rate, or extent of interleukin-19 production. Sources: GOC:mah Also known as: regulation of IL-19 production, regulation of interleukin-19 biosynthetic process Relationships: is a type of GO:0001817; regulates interleukin-19 production [GO:0032622] Subtypes: negative regulation of interleukin-19 production [GO:0032702], GO:0032742